trimethylamine monooxygenase activity [GO:0034899] (molecular function) Sources: EC:1.14.13.148, UM-BBD_reactionID:r1407 Definition: Catalysis of the reaction: N,N,N-trimethylamine + NADPH + H+ + O2 = N,N,N-trimethylamine N-oxide + NADP+ + H2O. Relationships: is a type of GO:0016709